regulation of B cell cytokine production [GO:0002721] (biological process) Definition: Any process that modulates the frequency, rate, or extent of B cell cytokine production. Relationships: is a type of GO:0002712; is a type of regulation of cytokine production involved in immune response [GO:0002718]; regulates B cell cytokine production [GO:0002368] Sources: GOC:add Also known as: regulation of B lymphocyte cytokine production, regulation of B-cell cytokine production, regulation of B-lymphocyte cytokine production Subtypes: GO:0002722, positive regulation of B cell cytokine production [GO:0002723]